{
  "gene_name": "Eukaryotic translation initiation factor 2-alpha kinase 3",
  "gene": "UniProtKB:Q9NZJ5",
  "term_id": "GO:0017148",
  "term_label": "negative regulation of translation",
  "gene_symbol": "EIF2AK3"
}